{
  "gene_symbol": "USP14",
  "term_id": "UNKNOWN:0003",
  "term_label": "Unknown cellular component",
  "gene_name": "Ubiquitin carboxyl-terminal hydrolase 14",
  "gene": "UniProtKB:P54578"
}